{
  "term_label": "early endosome",
  "gene": "UniProtKB:Q9Y4E1",
  "term_id": "GO:0005769",
  "gene_symbol": "WASHC2C",
  "gene_name": "WASH complex subunit 2C"
}